{
  "gene_symbol": "DGAT2L6",
  "gene_name": "Diacylglycerol O-acyltransferase 2-like protein 6",
  "gene": "UniProtKB:Q6ZPD8",
  "term_id": "GO:0005789",
  "term_label": "endoplasmic reticulum membrane"
}